{
  "term_id": "UNKNOWN:0001",
  "gene": "UniProtKB:Q5VIR6",
  "gene_name": "Vacuolar protein sorting-associated protein 53 homolog",
  "term_label": "Unknown molecular function",
  "gene_symbol": "VPS53"
}